{
  "term_label": "lipopolysaccharide binding",
  "gene_name": "Monocyte differentiation antigen CD14",
  "term_id": "GO:0001530",
  "gene_symbol": "CD14",
  "gene": "UniProtKB:P08571"
}